2-oxoglutarate-dependent dioxygenase activity [GO:0016706] (molecular function) Subtypes: GO:0000907, GO:0000908, GO:0008336, GO:0008475, GO:0016707, 2,4-dichlorophenoxyacetate alpha-ketoglutarate dioxygenase activity [GO:0018602], peptidyl-proline dioxygenase activity [GO:0031543], histone H3R2 demethylase activity [GO:0033746], GO:0033749, GO:0033758, flavone synthase activity [GO:0033759], GO:0033760, mugineic-acid 3-dioxygenase activity [GO:0033761], proline 3-hydroxylase activity [GO:0033763], histone H3K4me/H3K4me2/H3K4me3 demethylase activity [GO:0034647], oxidative RNA demethylase activity [GO:0035515], broad specificity oxidative DNA demethylase activity [GO:0035516], histone H4K20 demethylase activity [GO:0035575], peptidyl-histidine dioxygenase activity [GO:0036139], [protein]-asparagine 3-dioxygenase activity [GO:0036140], flavonol synthase activity [GO:0045431], deacetoxycephalosporin-C hydroxylase activity [GO:0045442], flavanone 3-dioxygenase activity [GO:0045486], GO:0045543, gibberellin 20-oxidase activity [GO:0045544], deoxyuridine 1'-dioxygenase activity [GO:0047079], deoxyuridine 2'-dioxygenase activity [GO:0047080], 6-beta-hydroxyhyoscyamine epoxidase activity [GO:0047594], hyoscyamine (6S)-dioxygenase activity [GO:0047998], phytanoyl-CoA dioxygenase activity [GO:0048244], thymine dioxygenase activity [GO:0050341], GO:0050353, leucocyanidin oxygenase activity [GO:0050589], desacetoxyvindoline 4-hydroxylase activity [GO:0050590], histone H3K36 demethylase activity [GO:0051864], peptidyl-aspartic acid 3-dioxygenase activity [GO:0062101], L-gamma-glutamyl-L-propargylglycine hydroxylase activity [GO:0062148], DNA 5-methylcytosine dioxygenase activity [GO:0070579], GO:0070815, GO:0071558, GO:0102312, tRNA(Phe) (7-(3-amino-3-carboxypropyl)wyosine37-C2)-hydroxylase activity [GO:0102524], 2-oxoglutarate, L-arginine oxygenase (succinate-forming) activity [GO:0102525], thebaine 6-O-demethylase activity [GO:0102802], codeine O-demethylase activity [GO:0102805], GO:0106155, peptidyl-lysine 4-dioxygenase activity [GO:0106156], GO:0106157, glutarate dioxygenase activity [GO:0106343], histone H3K9me/H3K9me2 demethylase activity [GO:0140683], GO:0140684, histone H3K56me2/H3K56me3 demethylase activity [GO:0140760], DNA N6-methyladenine demethylase activity [GO:0141131], 2-oxoglutarate-dependent tRNA 5-methylcytidine formyltransferase activity [GO:0160290] Sources: GOC:mah Definition: Catalysis of the reaction: A + 2-oxoglutarate + O2 = B + succinate + CO2. This is an oxidation-reduction (redox) reaction in which hydrogen or electrons are transferred from 2-oxoglutarate and one other donor, and one atom of oxygen is incorporated into each donor. Also known as: 2-oxoglutarate dioxygenase activity, oxidoreductase activity, acting on paired donors, with incorporation or reduction of molecular oxygen, 2-oxoglutarate as one donor, and incorporation of one atom each of oxygen into both donors Relationships: is_a GO:0016705; is a type of dioxygenase activity [GO:0051213]